{
  "term_id": "GO:0006865",
  "term_label": "amino acid transport",
  "gene": "UniProtKB:Q01959",
  "gene_name": "Sodium-dependent dopamine transporter",
  "gene_symbol": "SLC6A3"
}